N-acetylmannosamine metabolic process [GO:0006051] (biological process) Subtypes: N-acetylmannosamine biosynthetic process [GO:0006052], N-acetylmannosamine catabolic process [GO:0006053] Relationships: is a type of amino sugar metabolic process [GO:0006040] Definition: The chemical reactions and pathways involving N-acetylmannosamine, the acetylated derivative of mannosamine, 2-amino-2-deoxymannose. Also known as: N-acetylmannosamine metabolism Sources: GOC:ai, ISBN:0198506732